{
  "term_id": "GO:0007288",
  "gene_name": "Dynein regulatory complex protein 9",
  "gene": "UniProtKB:Q9H095",
  "gene_symbol": "IQCG",
  "term_label": "sperm axoneme assembly"
}